{
  "term_label": "endosome",
  "gene": "UniProtKB:Q96S21",
  "gene_name": "Ras-related protein Rab-40C",
  "gene_symbol": "RAB40C",
  "term_id": "GO:0005768"
}